{
  "gene_symbol": "CALR3",
  "term_id": "GO:0005789",
  "term_label": "endoplasmic reticulum membrane",
  "gene_name": "Calreticulin-3",
  "gene": "UniProtKB:Q96L12"
}